cellulose 1,4-beta-cellobiosidase activity [GO:0016162] (molecular function) Sources: EC:3.2.1.91 Relationships: is a type of GO:0004553 Also known as: avicelase activity, 1,4-beta-D-glucan cellobiohydrolase activity, 1,4-beta-cellobiohydrolase activity, 1,4-beta-glucan cellobiosidase activity, C1 cellulase activity, CBH 1, beta-1,4-glucan cellobiohydrolase activity, beta-1,4-glucan cellobiosylhydrolase activity, cellobiohydrolase I, cellobiohydrolase activity, cellobiosidase activity, exo-1,4-beta-D-glucanase activity, exo-beta-1,4-glucan cellobiohydrolase activity, exo-cellobiohydrolase activity, exocellobiohydrolase activity, exoglucanase activity Definition: Catalysis of the hydrolysis of (1->4)-beta-D-glucosidic linkages in cellulose and cellotetraose, releasing cellobiose from the non-reducing ends of the chains.